{
  "gene_name": "Short-chain dehydrogenase_reductase family 42E member 1",
  "gene": "UniProtKB:Q8WUS8",
  "gene_symbol": "SDR42E1",
  "term_label": "Unknown cellular component",
  "term_id": "UNKNOWN:0003"
}